glucose homeostasis [GO:0042593] (biological process) Sources: GOC:go_curators Definition: Any process involved in the maintenance of an internal steady state of glucose within an organism or cell. Subtypes: intracellular glucose homeostasis [GO:0001678] Relationships: is a type of carbohydrate homeostasis [GO:0033500]